regulation of transcription elongation by RNA polymerase II [GO:0034243] (biological process) Sources: GOC:mah, GOC:txnOH Definition: Any process that modulates the frequency, rate or extent of transcription elongation, the extension of an RNA molecule after transcription initiation and promoter clearance by the addition of ribonucleotides, catalyzed by RNA polymerase II. Also known as: regulation of RNA elongation from RNA polymerase II promoter, regulation of transcription elongation from RNA polymerase II promoter, regulation of gene-specific transcription elongation from RNA polymerase II promoter Relationships: is a type of regulation of DNA-templated transcription elongation [GO:0032784]; regulates transcription elongation by RNA polymerase II [GO:0006368] Subtypes: positive regulation of transcription elongation by RNA polymerase II [GO:0032968], negative regulation of transcription elongation by RNA polymerase II [GO:0034244]